{
  "term_label": "Unknown biological process",
  "gene_symbol": "XK",
  "gene_name": "Endoplasmic reticulum membrane adapter protein XK",
  "term_id": "UNKNOWN:0002",
  "gene": "UniProtKB:P51811"
}